{
  "term_id": "GO:0005634",
  "term_label": "nucleus",
  "gene_symbol": "DDX51",
  "gene_name": "ATP-dependent RNA helicase DDX51",
  "gene": "UniProtKB:Q8N8A6"
}